pyrimidine nucleoside salvage [GO:0043097] (biological process) Sources: GOC:jl Subtypes: pyrimidine deoxyribonucleoside salvage [GO:0043099] Relationships: is a type of pyrimidine-containing compound salvage [GO:0008655]; is a type of nucleoside salvage [GO:0043174]; is a type of pyrimidine nucleoside biosynthetic process [GO:0046134] Definition: Any process that generates a pyrimidine nucleoside, one of a family of organic molecules consisting of a pyrimidine base covalently bonded to a sugar ribose, from derivatives of it, without de novo synthesis.